{
  "gene_name": "LON peptidase N-terminal domain and RING finger protein 1",
  "gene_symbol": "LONRF1",
  "gene": "UniProtKB:Q17RB8",
  "term_label": "Unknown cellular component",
  "term_id": "UNKNOWN:0003"
}